{
  "gene_symbol": "ZBTB8B",
  "term_id": "GO:0000981",
  "gene": "UniProtKB:Q8NAP8",
  "term_label": "DNA-binding transcription factor activity, RNA polymerase II-specific",
  "gene_name": "Zinc finger and BTB domain-containing protein 8B"
}